{
  "gene": "UniProtKB:Q9Y227",
  "gene_symbol": "ENTPD4",
  "gene_name": "Ectonucleoside triphosphate diphosphohydrolase 4",
  "term_id": "GO:0016020",
  "term_label": "membrane"
}